{
  "gene": "UniProtKB:Q8IXK0",
  "gene_symbol": "PHC2",
  "term_label": "histone binding",
  "gene_name": "Polyhomeotic-like protein 2",
  "term_id": "GO:0042393"
}